{
  "term_id": "UNKNOWN:0002",
  "gene_symbol": "KNCN",
  "term_label": "Unknown biological process",
  "gene_name": "Kinocilin",
  "gene": "UniProtKB:A6PVL3"
}